{
  "term_id": "UNKNOWN:0002",
  "gene_symbol": "RBM48",
  "term_label": "Unknown biological process",
  "gene": "UniProtKB:Q5RL73",
  "gene_name": "RNA-binding protein 48"
}